{
  "gene_symbol": "HELQ",
  "term_id": "GO:0045003",
  "gene_name": "Helicase POLQ-like",
  "term_label": "double-strand break repair via synthesis-dependent strand annealing",
  "gene": "UniProtKB:Q8TDG4"
}